{
  "gene_symbol": "FBH1",
  "gene_name": "F-box DNA helicase 1",
  "term_label": "nucleus",
  "gene": "UniProtKB:Q8NFZ0",
  "term_id": "GO:0005634"
}